{
  "term_id": "GO:0005886",
  "term_label": "plasma membrane",
  "gene": "UniProtKB:Q8NGN7",
  "gene_name": "Putative olfactory receptor 10D4",
  "gene_symbol": "OR10D4P"
}